{
  "term_label": "Unknown molecular function",
  "gene_name": "Transmembrane and coiled-coil domain-containing protein 3",
  "gene": "UniProtKB:Q6UWJ1",
  "gene_symbol": "TMCO3",
  "term_id": "UNKNOWN:0001"
}